{
  "term_label": "cytosol",
  "gene": "UniProtKB:P14735",
  "gene_symbol": "IDE",
  "term_id": "GO:0005829",
  "gene_name": "Insulin-degrading enzyme"
}